{
  "term_id": "GO:0007155",
  "term_label": "cell adhesion",
  "gene": "UniProtKB:P20908",
  "gene_symbol": "COL5A1",
  "gene_name": "Collagen alpha-1(V) chain"
}